{
  "gene_symbol": "AGTPBP1",
  "term_label": "metallocarboxypeptidase activity",
  "term_id": "GO:0004181",
  "gene": "UniProtKB:Q9UPW5",
  "gene_name": "Cytosolic carboxypeptidase 1"
}